{
  "gene_name": "Radial spoke head 10 homolog B",
  "term_label": "Unknown biological process",
  "gene": "UniProtKB:P0C881",
  "term_id": "UNKNOWN:0002",
  "gene_symbol": "RSPH10B"
}